{
  "term_label": "Unknown molecular function",
  "term_id": "UNKNOWN:0001",
  "gene": "UniProtKB:Q96ND0",
  "gene_symbol": "FAM210A",
  "gene_name": "Protein FAM210A"
}